{
  "gene_name": "Tripartite motif-containing protein 42",
  "term_id": "UNKNOWN:0002",
  "term_label": "Unknown biological process",
  "gene": "UniProtKB:Q8IWZ5",
  "gene_symbol": "TRIM42"
}